{
  "gene_symbol": "IGLV1-47",
  "gene_name": "Immunoglobulin lambda variable 1-47",
  "term_id": "GO:0006955",
  "gene": "UniProtKB:P01700",
  "term_label": "immune response"
}